glucose sensor activity [GO:0141089] (MF) Relationships: is a type of molecular sensor activity [GO:0140299]; has part D-glucose binding [GO:0005536] Also known as: glucose sensing activity References: PMID:17470517 Definition: Binding to and responding, e.g. by conformational change, to changes in the cellular level of glucose.